{
  "gene_symbol": "STX6",
  "term_label": "endomembrane system",
  "term_id": "GO:0012505",
  "gene_name": "Syntaxin-6",
  "gene": "UniProtKB:O43752"
}